{
  "term_id": "GO:0017116",
  "term_label": "single-stranded DNA helicase activity",
  "gene_name": "Helicase POLQ-like",
  "gene": "UniProtKB:Q8TDG4",
  "gene_symbol": "HELQ"
}